oxygen transport [GO:0015671] (BP) Definition: The directed movement of oxygen (O2) into, out of or within a cell, or between cells, by means of some agent such as a transporter or pore. Sources: GOC:ai Relationships: is a type of gas transport [GO:0015669]